{
  "gene": "UniProtKB:Q8IZ57",
  "gene_symbol": "NRSN1",
  "term_id": "GO:0030133",
  "term_label": "transport vesicle",
  "gene_name": "Neurensin-1"
}